{
  "term_label": "receptor-mediated endocytosis",
  "term_id": "GO:0006898",
  "gene": "UniProtKB:O75165",
  "gene_name": "DnaJ homolog subfamily C member 13",
  "gene_symbol": "DNAJC13"
}